response to caloric restriction [GO:0061771] (BP) Subtypes: cellular response to caloric restriction [GO:0061433] Relationships: is a type of response to stress [GO:0006950]; is a type of response to nutrient levels [GO:0031667] References: PMID:15520862 Sources: GOC:dph Definition: A change in state or activity of a cell or an organism (in terms of movement, secretion, enzyme production, gene expression, etc.) as a result of a caloric restriction, insufficient food energy intake.